{
  "gene_name": "Trichohyalin-like protein 1",
  "term_id": "UNKNOWN:0003",
  "gene_symbol": "TCHHL1",
  "term_label": "Unknown cellular component",
  "gene": "UniProtKB:Q5QJ38"
}